{
  "gene_name": "G1_S-specific cyclin-E1",
  "gene": "UniProtKB:P24864",
  "gene_symbol": "CCNE1",
  "term_label": "microtubule organizing center",
  "term_id": "GO:0005815"
}